{
  "gene": "UniProtKB:P06133",
  "gene_name": "UDP-glucuronosyltransferase 2B4",
  "term_label": "glucuronosyltransferase activity",
  "term_id": "GO:0015020",
  "gene_symbol": "UGT2B4"
}